{
  "term_id": "UNKNOWN:0001",
  "gene": "UniProtKB:A6NFE3",
  "term_label": "Unknown molecular function",
  "gene_symbol": "EFCAB10",
  "gene_name": "EF-hand calcium-binding domain-containing protein 10"
}